{
  "term_label": "cytosol",
  "term_id": "GO:0005829",
  "gene": "UniProtKB:Q9H1P3",
  "gene_symbol": "OSBPL2",
  "gene_name": "Oxysterol-binding protein-related protein 2"
}